{
  "gene": "UniProtKB:Q2KHR2",
  "term_label": "regulation of transcription by RNA polymerase II",
  "gene_symbol": "RFX7",
  "term_id": "GO:0006357",
  "gene_name": "DNA-binding protein RFX7"
}